{
  "term_label": "regulation of gene expression",
  "gene_name": "Lysine-specific demethylase 6A",
  "term_id": "GO:0010468",
  "gene": "UniProtKB:O15550",
  "gene_symbol": "KDM6A"
}